{
  "term_label": "nucleus",
  "gene_name": "Splicing regulator SDE2",
  "term_id": "GO:0005634",
  "gene": "UniProtKB:Q6IQ49",
  "gene_symbol": "SDE2"
}